{
  "gene_name": "Integral membrane protein GPR137C",
  "term_id": "GO:0005765",
  "gene_symbol": "GPR137C",
  "term_label": "lysosomal membrane",
  "gene": "UniProtKB:Q8N3F9"
}